{
  "term_id": "GO:0032580",
  "gene_symbol": "GOLGA8O",
  "gene": "UniProtKB:A6NCC3",
  "term_label": "Golgi cisterna membrane",
  "gene_name": "Golgin subfamily A member 8O"
}